{
  "term_label": "protein-RNA complex assembly",
  "gene_name": "Large ribosomal subunit protein eL38",
  "term_id": "GO:0022618",
  "gene": "UniProtKB:P63173",
  "gene_symbol": "RPL38"
}